5alpha,9alpha,10beta-labda-8(20),13-dien-15-yl diphosphate catabolic process [GO:1901948] (biological process) References: PMID:22027823 Sources: GOC:TermGenie Relationships: is a type of phospholipid catabolic process [GO:0009395]; is a type of diterpenoid catabolic process [GO:0016103] Definition: The chemical reactions and pathways resulting in the breakdown of 5alpha,9alpha,10beta-labda-8(20),13-dien-15-yl diphosphate. Also known as: 5alpha,9alpha,10beta-labda-8(20),13-dien-15-yl diphosphate breakdown, 5alpha,9alpha,10beta-labda-8(20),13-dien-15-yl diphosphate catabolism, 5alpha,9alpha,10beta-labda-8(20),13-dien-15-yl diphosphate degradation